{
  "term_id": "GO:0005634",
  "gene_symbol": "ZNF513",
  "gene_name": "Zinc finger protein 513",
  "gene": "UniProtKB:Q8N8E2",
  "term_label": "nucleus"
}